{
  "gene_symbol": "GPR37L1",
  "term_label": "plasma membrane",
  "gene_name": "G-protein coupled receptor 37-like 1",
  "gene": "UniProtKB:O60883",
  "term_id": "GO:0005886"
}